{
  "term_label": "positive regulation of MAPK cascade",
  "gene_name": "Fibroblast growth factor 20",
  "gene": "UniProtKB:Q9NP95",
  "term_id": "GO:0043410",
  "gene_symbol": "FGF20"
}